{
  "term_label": "calcium channel regulator activity",
  "gene_symbol": "CABP1",
  "gene_name": "Calcium-binding protein 1",
  "term_id": "GO:0005246",
  "gene": "UniProtKB:Q9NZU7"
}